ciliary centrin arm assembly [GO:0120273] (biological process) Definition: The aggregation, arrangement and bonding together of a set of macromolecules to form a ciliary centrin arm, a rod-shaped protein complex containing Centrin4 protein that flanks the flagellum attachment zone (FAZ) filament and the quartet microtubules. Also known as: ciliary centrin arm formation Relationships: is a type of protein-containing complex assembly [GO:0065003]; is part of cilium assembly [GO:0060271] References: PMID:32675283 Sources: GOC:ach, GOC:krc